{
  "gene": "UniProtKB:P08684",
  "gene_symbol": "CYP3A4",
  "term_id": "GO:0008202",
  "gene_name": "Cytochrome P450 3A4",
  "term_label": "steroid metabolic process"
}